regulation of response to toluene [GO:1901454] (BP) Sources: GOC:TermGenie, GOC:mengo_curators Relationships: is a type of regulation of response to stimulus [GO:0048583]; RO_0002211 response to toluene [GO:1901424] Subtypes: negative regulation of response to toluene [GO:1901455], positive regulation of response to toluene [GO:1901456] Definition: Any process that modulates the frequency, rate or extent of response to toluene.